{
  "term_label": "Unknown cellular component",
  "gene": "UniProtKB:A2A3L6",
  "term_id": "UNKNOWN:0003",
  "gene_name": "Tetratricopeptide repeat protein 24",
  "gene_symbol": "TTC24"
}